{
  "gene": "UniProtKB:O15247",
  "term_id": "GO:0016020",
  "gene_symbol": "CLIC2",
  "term_label": "membrane",
  "gene_name": "Chloride intracellular channel protein 2"
}